{
  "gene_symbol": "DUXA",
  "term_id": "GO:0000977",
  "term_label": "RNA polymerase II transcription regulatory region sequence-specific DNA binding",
  "gene_name": "Double homeobox protein A",
  "gene": "UniProtKB:A6NLW8"
}